{
  "term_label": "activin receptor signaling pathway",
  "gene_symbol": "TGFBR1",
  "gene_name": "TGF-beta receptor type-1",
  "gene": "UniProtKB:P36897",
  "term_id": "GO:0032924"
}